{
  "term_label": "Unknown biological process",
  "gene_symbol": "CHADL",
  "gene": "UniProtKB:Q6NUI6",
  "term_id": "UNKNOWN:0002",
  "gene_name": "Chondroadherin-like protein"
}